regulation of postsynaptic membrane organization [GO:1901626] (biological process) Definition: Any process that modulates the frequency, rate or extent of postsynaptic membrane organization. References: PMID:22426000 Sources: GOC:TermGenie Also known as: regulation of post-synaptic membrane organization, regulation of postsynaptic membrane organisation Relationships: is a type of regulation of cellular component organization [GO:0051128]; regulates GO:0001941 Subtypes: negative regulation of postsynaptic membrane organization [GO:1901627], positive regulation of postsynaptic membrane organization [GO:1901628]